{
  "gene": "UniProtKB:P78539",
  "gene_name": "Sushi repeat-containing protein SRPX",
  "gene_symbol": "SRPX",
  "term_id": "UNKNOWN:0003",
  "term_label": "Unknown cellular component"
}